{
  "gene": "UniProtKB:Q15672",
  "gene_symbol": "TWIST1",
  "term_id": "GO:0006357",
  "term_label": "regulation of transcription by RNA polymerase II",
  "gene_name": "Twist-related protein 1"
}